{
  "term_label": "focal adhesion",
  "gene": "UniProtKB:P56945",
  "gene_symbol": "BCAR1",
  "gene_name": "Breast cancer anti-estrogen resistance protein 1",
  "term_id": "GO:0005925"
}